{
  "term_label": "nucleus",
  "gene": "UniProtKB:Q8IZL8",
  "gene_name": "Proline-, glutamic acid- and leucine-rich protein 1",
  "gene_symbol": "PELP1",
  "term_id": "GO:0005634"
}